'de novo' XMP biosynthetic process [GO:0097294] (biological process) Definition: The chemical reactions and pathways resulting in the formation of XMP, xanthosine monophosphate, from simpler precursors. Relationships: is a type of GO:0097293 References: PMID:27590927 Sources: GOC:yaf Also known as: 'de novo' XMP anabolism, 'de novo' XMP biosynthesis, 'de novo' XMP formation, 'de novo' XMP synthesis